{
  "gene_name": "Integrin beta-2",
  "gene_symbol": "ITGB2",
  "gene": "UniProtKB:P05107",
  "term_id": "GO:0033627",
  "term_label": "cell adhesion mediated by integrin"
}